{
  "gene_symbol": "TMEM74B",
  "gene_name": "Transmembrane protein 74B",
  "term_label": "Unknown biological process",
  "term_id": "UNKNOWN:0002",
  "gene": "UniProtKB:Q9NUR3"
}